hydroxylysine catabolic process [GO:0046948] (biological process) Definition: The chemical reactions and pathways resulting in the breakdown of hydroxylysine (5-hydroxy-2,6-diaminohexanoic acid), a chiral alpha-amino acid. Also known as: hydroxylysine breakdown, hydroxylysine catabolism, hydroxylysine degradation Relationships: is a type of modified amino acid catabolic process [GO:0042219]; is a type of non-proteinogenic amino acid catabolic process [GO:0170044]; is a type of alpha-amino acid catabolic process [GO:1901606] Sources: ISBN:0198506732